{
  "term_id": "GO:0005634",
  "gene": "UniProtKB:Q7L945",
  "term_label": "nucleus",
  "gene_symbol": "ZNF627",
  "gene_name": "Zinc finger protein 627"
}